{
  "gene_symbol": "APPBP2",
  "term_id": "GO:0043161",
  "term_label": "proteasome-mediated ubiquitin-dependent protein catabolic process",
  "gene_name": "Amyloid protein-binding protein 2",
  "gene": "UniProtKB:Q92624"
}